positive regulation of glial cell-derived neurotrophic factor production [GO:1900168] (biological process) Also known as: positive regulation of GDNF production, activation of glial cell line-derived neurotrophic factor secretion, positive regulation of glial cell-derived neurotrophic factor secretion, positive regulation of glial cell line-derived neurotrophic factor secretion Sources: GOC:TermGenie, GOC:yaf Relationships: is a type of positive regulation of cytokine production [GO:0001819]; is_a GO:1900166; positively regulates glial cell-derived neurotrophic factor production [GO:0044467] Definition: Any process that activates or increases the frequency, rate or extent of glial cell-derived neurotrophic factor production.